{
  "term_id": "GO:1990756",
  "term_label": "ubiquitin-like ligase-substrate adaptor activity",
  "gene_symbol": "KLHL9",
  "gene": "UniProtKB:Q9P2J3",
  "gene_name": "Kelch-like protein 9"
}